{
  "term_id": "GO:0015629",
  "gene_symbol": "MTSS2",
  "gene": "UniProtKB:Q765P7",
  "term_label": "actin cytoskeleton",
  "gene_name": "Protein MTSS 2"
}